1-aminocyclopropane-1-carboxylate metabolic process [GO:0018871] (biological process) Regulation: regulated by regulation of 1-aminocyclopropane-1-carboxylate metabolic process [GO:0010602] Also known as: 1-aminocyclopropane-1-carboxylate metabolism, ACP metabolic process, ACP metabolism Subtypes: GO:0042217, 1-aminocyclopropane-1-carboxylate biosynthetic process [GO:0042218] Sources: UM-BBD_pathwayID:acp Definition: The chemical reactions and pathways involving 1-aminocyclopropane-1-carboxylate, the anion of 1-aminocyclopropane-1-carboxylic acid, a natural product found in plant tissues. It is a key intermediate in the biosynthesis of ethylene (ethene), a fruit-ripening hormone in plants. Relationships: is a type of non-proteinogenic amino acid metabolic process [GO:0170041]; is a type of alpha-amino acid metabolic process [GO:1901605]